peptidyl-histidine dephosphorylation [GO:0035971] (biological process) Definition: The removal of phosphoric residues from peptidyl-O-phospho-L-histidine to form peptidyl-histidine. References: PMID:12383260 Sources: GOC:BHF, GOC:vk Relationships: is_a GO:0006470